regulation of lymphoid progenitor cell differentiation [GO:1905456] (biological process) Definition: Any process that modulates the frequency, rate or extent of lymphoid progenitor cell differentiation. References: PMID:27010503 Sources: GOC:TermGenie, GO_REF:0000058 Relationships: is a type of regulation of hematopoietic progenitor cell differentiation [GO:1901532]; regulates lymphoid progenitor cell differentiation [GO:0002320] Subtypes: negative regulation of lymphoid progenitor cell differentiation [GO:1905457], positive regulation of lymphoid progenitor cell differentiation [GO:1905458], regulation of pro-T cell differentiation [GO:2000174], GO:2000973